{
  "gene_symbol": "NDUFA5",
  "term_id": "GO:0022904",
  "gene_name": "NADH dehydrogenase [ubiquinone] 1 alpha subcomplex subunit 5",
  "gene": "UniProtKB:Q16718",
  "term_label": "respiratory electron transport chain"
}